{
  "gene_name": "AP-3 complex subunit delta-1",
  "gene": "UniProtKB:O14617",
  "gene_symbol": "AP3D1",
  "term_label": "protein targeting to vacuole",
  "term_id": "GO:0006623"
}